glycerol metabolic process [GO:0006071] (biological process) Sources: GOC:ai, ISBN:0198506732 Relationships: is a type of carbohydrate metabolic process [GO:0005975]; is a type of polyol metabolic process [GO:0019751] Subtypes: GO:0006114, glycerol catabolic process [GO:0019563], glycerol to glycerone phosphate metabolic process [GO:0061610] Also known as: glycerol metabolism Definition: The chemical reactions and pathways involving glycerol, 1,2,3-propanetriol, a sweet, hygroscopic, viscous liquid, widely distributed in nature as a constituent of many lipids.